{
  "term_label": "positive regulation of osteoblast differentiation",
  "gene": "UniProtKB:P55107",
  "term_id": "GO:0045669",
  "gene_name": "Growth_differentiation factor 10",
  "gene_symbol": "GDF10"
}